{
  "term_id": "GO:0000981",
  "gene": "UniProtKB:Q06413",
  "term_label": "DNA-binding transcription factor activity, RNA polymerase II-specific",
  "gene_name": "Myocyte-specific enhancer factor 2C",
  "gene_symbol": "MEF2C"
}